{
  "gene": "UniProtKB:Q05D60",
  "gene_symbol": "DEUP1",
  "term_id": "GO:0098535",
  "term_label": "de novo centriole assembly involved in multi-ciliated epithelial cell differentiation",
  "gene_name": "Deuterosome assembly protein 1"
}